{
  "gene_name": "NTF2-related export protein 2",
  "gene_symbol": "NXT2",
  "term_id": "GO:0016973",
  "gene": "UniProtKB:Q9NPJ8",
  "term_label": "poly(A)+ mRNA export from nucleus"
}